{
  "gene_symbol": "SHANK1",
  "gene_name": "SH3 and multiple ankyrin repeat domains protein 1",
  "term_id": "GO:0008306",
  "gene": "UniProtKB:Q9Y566",
  "term_label": "associative learning"
}